{
  "term_id": "GO:0097039",
  "gene": "UniProtKB:Q9BYM8",
  "term_label": "protein linear polyubiquitination",
  "gene_symbol": "RBCK1",
  "gene_name": "RanBP-type and C3HC4-type zinc finger-containing protein 1"
}